{
  "term_label": "carboxylic acid transmembrane transport",
  "gene": "UniProtKB:O15374",
  "term_id": "GO:1905039",
  "gene_symbol": "SLC16A4",
  "gene_name": "Monocarboxylate transporter 5"
}